{
  "gene": "UniProtKB:A6NK59",
  "term_id": "UNKNOWN:0003",
  "term_label": "Unknown cellular component",
  "gene_name": "Ankyrin repeat and SOCS box protein 14",
  "gene_symbol": "ASB14"
}